intracellular phosphate ion homeostasis [GO:0030643] (biological process) Also known as: intracellular phosphate homeostasis, cellular phosphate ion homeostasis, intracellular Pi homeostasis Sources: GOC:mah Relationships: is a type of phosphate ion homeostasis [GO:0055062]; is a type of intracellular chemical homeostasis [GO:0055082] Definition: A homeostatic process involved in the maintenance of a steady state level of phosphate ions within a cell.